beta-ketodecanoyl-[acyl-carrier-protein] synthase activity [GO:0061990] (molecular function) Definition: Catalysis of the reaction: octanoyl-CoA + H+ + malonyl-[ACP] = 3-oxodecanoyl-[ACP] + CO2 + CoA. References: PMID:22753057 Sources: RHEA:42264 Relationships: is_a GO:0016747